{
  "gene": "UniProtKB:C9J202",
  "gene_name": "Putative glycosyltransferase ALG1L2",
  "term_id": "UNKNOWN:0002",
  "gene_symbol": "ALG1L2",
  "term_label": "Unknown biological process"
}